{
  "gene": "UniProtKB:Q9BX66",
  "gene_symbol": "SORBS1",
  "gene_name": "Sorbin and SH3 domain-containing protein 1",
  "term_label": "signaling receptor complex adaptor activity",
  "term_id": "GO:0030159"
}